{
  "gene_symbol": "OR11H7",
  "gene": "UniProtKB:Q8NGC8",
  "term_label": "Unknown biological process",
  "term_id": "UNKNOWN:0002",
  "gene_name": "Olfactory receptor 11H7"
}